{
  "gene_symbol": "SRSF11",
  "gene": "UniProtKB:Q05519",
  "gene_name": "Serine_arginine-rich splicing factor 11",
  "term_label": "Unknown biological process",
  "term_id": "UNKNOWN:0002"
}